{
  "gene_name": "RAB11-binding protein RELCH",
  "gene": "UniProtKB:Q9P260",
  "term_id": "UNKNOWN:0001",
  "gene_symbol": "RELCH",
  "term_label": "Unknown molecular function"
}